{
  "gene_symbol": "CD248",
  "term_id": "GO:1990430",
  "gene": "UniProtKB:Q9HCU0",
  "gene_name": "Endosialin",
  "term_label": "extracellular matrix protein binding"
}